{
  "gene": "UniProtKB:Q8NFA2",
  "term_label": "superoxide anion generation",
  "term_id": "GO:0042554",
  "gene_name": "NADPH oxidase organizer 1",
  "gene_symbol": "NOXO1"
}